regulation of eukaryotic translation initiation factor 4F complex assembly [GO:1905535] (BP) Also known as: regulation of eIF-4F assembly, regulation of eIF4F assembly Subtypes: negative regulation of eukaryotic translation initiation factor 4F complex assembly [GO:1905536], positive regulation of eukaryotic translation initiation factor 4F complex assembly [GO:1905537] Relationships: is a type of GO:0043254; regulates GO:0097010 Definition: Any process that modulates the frequency, rate or extent of eukaryotic translation initiation factor 4F complex assembly. References: PMID:18426977 Sources: GOC:PARL, GOC:TermGenie, GOC:bc, GO_REF:0000058